fibrinolysis [GO:0042730] (biological process) Definition: A process that solubilizes fibrin in the bloodstream of a multicellular organism, chiefly by the proteolytic action of plasmin. Regulation: regulated by regulation of fibrinolysis [GO:0051917]; RO_0002212 by negative regulation of fibrinolysis [GO:0051918]; positively regulated by positive regulation of fibrinolysis [GO:0051919] References: PMID:15842654 Sources: GOC:jl Relationships: is a type of GO:0030195